{
  "gene": "UniProtKB:P26640",
  "term_id": "GO:0006438",
  "gene_symbol": "VARS1",
  "gene_name": "Valine--tRNA ligase",
  "term_label": "valyl-tRNA aminoacylation"
}